{
  "term_id": "GO:0038023",
  "gene_symbol": "ITGA4",
  "gene": "UniProtKB:P13612",
  "term_label": "signaling receptor activity",
  "gene_name": "Integrin alpha-4"
}